quinone binding [GO:0048038] (molecular function) Definition: Binding to a quinone, any member of a class of diketones derivable from aromatic compounds by conversion of two CH groups into CO groups with any necessary rearrangement of double bonds. Sources: ISBN:0198506732 Relationships: is a type of small molecule binding [GO:0036094] Subtypes: GO:0048039